positive regulation of iron ion import across plasma membrane [GO:1904440] (BP) Relationships: is a type of GO:0034761; is a type of regulation of iron ion import across plasma membrane [GO:1904438]; positively regulates iron ion import across plasma membrane [GO:0098711] Also known as: activation of ferrous ion import into cell, activation of ferrous iron import across plasma membrane, positive regulation of ferrous ion import into cell, positive regulation of ferrous iron import across plasma membrane, positive regulation of ferrous iron import into cell, up regulation of ferrous ion import into cell, up regulation of ferrous iron import across plasma membrane, up-regulation of ferrous ion import into cell, up-regulation of ferrous iron import across plasma membrane, upregulation of ferrous ion import into cell, upregulation of ferrous iron import across plasma membrane Definition: Any process that activates or increases the frequency, rate or extent of iron ions import across plasma membrane. References: PMID:18353247 Sources: GOC:BHF, GOC:TermGenie, GOC:kom, GO_REF:0000058